{
  "term_label": "Unknown molecular function",
  "gene_symbol": "KERA",
  "gene_name": "Keratocan",
  "gene": "UniProtKB:O60938",
  "term_id": "UNKNOWN:0001"
}